positive regulation of response to ethanol [GO:1901418] (BP) Definition: Any process that activates or increases the frequency, rate or extent of response to ethanol. Also known as: up regulation of response to ethanol, up-regulation of response to ethanol, upregulation of response to ethanol, activation of response to ethanol Sources: GOC:TermGenie, GOC:mengo_curators Relationships: is a type of regulation of response to ethanol [GO:1901416]; is a type of positive regulation of response to alcohol [GO:1901421]; positively regulates response to ethanol [GO:0045471]